{
  "gene_name": "Annexin A1",
  "gene": "UniProtKB:P04083",
  "gene_symbol": "ANXA1",
  "term_id": "GO:0007165",
  "term_label": "signal transduction"
}